{
  "gene_symbol": "TIPRL",
  "gene": "UniProtKB:O75663",
  "gene_name": "TIP41-like protein",
  "term_id": "GO:0031929",
  "term_label": "TOR signaling"
}